{
  "gene_name": "Protein FAM246A",
  "gene": "UniProtKB:A0A494C0Y3",
  "gene_symbol": "FAM246A",
  "term_id": "UNKNOWN:0002",
  "term_label": "Unknown biological process"
}